clathrin coat assembly [GO:0048268] (biological process) Definition: The process that results in the assembly of clathrin triskelia into the ordered structure known as a clathrin cage. Relationships: is a type of protein-containing complex assembly [GO:0065003] References: PMID:11460887, PMID:11977118, PMID:9531549 Sources: GOC:jid Subtypes: clathrin coating of Golgi vesicle [GO:0048202], clathrin coat assembly involved in endocytosis [GO:0099049] Regulation: regulated by regulation of clathrin coat assembly [GO:1905443]; negatively regulated by GO:1905444; positively regulated by positive regulation of clathrin coat assembly [GO:1905445] Also known as: clathrin cage assembly